male analia morphogenesis [GO:0048811] (biological process) References: PMID:11494318 Sources: GOC:mtg_sensu Definition: The process in which the anatomical structures of the analia of the male are generated and organized. The analia is the posterior-most vertral appendage that develops from the genital disc. Relationships: is a type of GO:0048809; is part of GO:0045496